{
  "gene": "UniProtKB:Q6IPT2",
  "gene_symbol": "GARIN5A",
  "gene_name": "Golgi-associated RAB2 interactor protein 5A",
  "term_label": "Unknown cellular component",
  "term_id": "UNKNOWN:0003"
}